{
  "gene_name": "Sestrin-2",
  "gene": "UniProtKB:P58004",
  "term_label": "cellular response to leucine starvation",
  "term_id": "GO:1990253",
  "gene_symbol": "SESN2"
}